{
  "gene": "UniProtKB:Q5TBK1",
  "term_id": "UNKNOWN:0002",
  "gene_name": "NEDD4-binding protein 2-like 1",
  "gene_symbol": "N4BP2L1",
  "term_label": "Unknown biological process"
}